cardioblast proliferation [GO:0003263] (biological process) Sources: GOC:mtg_heart Relationships: is_a GO:0061323; is part of heart formation [GO:0060914] Regulation: regulated by regulation of cardioblast proliferation [GO:0003264]; negatively regulated by negative regulation of cardioblast proliferation [GO:1905061]; positively regulated by GO:1905062 Definition: The multiplication or reproduction of cardioblasts, resulting in the expansion of the population in the heart field. A cardioblast is a cardiac precursor cell. It is a cell that has been committed to a cardiac fate, but will undergo more cell division rather than terminally differentiating.